{
  "gene_symbol": "TPBGL",
  "term_id": "GO:0005886",
  "gene": "UniProtKB:P0DKB5",
  "term_label": "plasma membrane",
  "gene_name": "Trophoblast glycoprotein-like"
}